endoderm development [GO:0007492] (biological process) Definition: The process whose specific outcome is the progression of the endoderm over time, from its formation to the mature structure. The endoderm is the innermost germ layer that develops into the gastrointestinal tract, the lungs and associated tissues. Sources: GOC:dph, GOC:tb Relationships: is a type of tissue development [GO:0009888]